{
  "term_id": "GO:0016020",
  "gene_name": "Putative fatty acid desaturase 2-like protein FADS2B",
  "term_label": "membrane",
  "gene": "UniProtKB:A8MWK0",
  "gene_symbol": "FADS2B"
}